{
  "term_label": "Unknown molecular function",
  "gene_name": "Coiled-coil domain-containing protein 77",
  "gene_symbol": "CCDC77",
  "term_id": "UNKNOWN:0001",
  "gene": "UniProtKB:Q9BR77"
}